{
  "gene_name": "Putative histone H2B type 2-D",
  "term_id": "GO:0030527",
  "term_label": "structural constituent of chromatin",
  "gene": "UniProtKB:Q6DRA6",
  "gene_symbol": "H2BC19P"
}